{
  "gene": "UniProtKB:Q8WVZ7",
  "term_label": "late endosome",
  "gene_symbol": "RNF133",
  "term_id": "GO:0005770",
  "gene_name": "E3 ubiquitin-protein ligase RNF133"
}